establishment of synaptic specificity at neuromuscular junction [GO:0007529] (biological process) Definition: The biological process in which a synapse between a motor neuron and a muscle is initially formed. Relationships: is a type of synapse organization [GO:0050808]; is part of neuromuscular junction development [GO:0007528] Sources: GOC:isa_complete